{
  "gene": "UniProtKB:A0A2R8Y4Y8",
  "gene_name": "Oocyte-secreted protein 4B",
  "term_id": "UNKNOWN:0003",
  "gene_symbol": "OOSP4B",
  "term_label": "Unknown cellular component"
}